large ribosomal subunit [GO:0015934] (cellular component) Subtypes: GO:0000315, GO:0022625 Sources: ISBN:0198506732 Relationships: is a type of ribosomal subunit [GO:0044391] Also known as: ribosomal large subunit Definition: The larger of the two subunits of a ribosome. Two sites on the ribosomal large subunit are involved in translation, namely the aminoacyl site (A site) and peptidyl site (P site).